{
  "gene": "UniProtKB:Q8WYQ4",
  "gene_name": "Uncharacterized protein C22orf15",
  "gene_symbol": "C22orf15",
  "term_label": "Unknown molecular function",
  "term_id": "UNKNOWN:0001"
}